{
  "term_id": "UNKNOWN:0001",
  "term_label": "Unknown molecular function",
  "gene": "UniProtKB:Q9ULG3",
  "gene_name": "Uncharacterized protein CFAP92",
  "gene_symbol": "CFAP92"
}